{
  "term_label": "scavenger receptor activity",
  "gene_symbol": "CD163",
  "gene": "UniProtKB:Q86VB7",
  "term_id": "GO:0005044",
  "gene_name": "Scavenger receptor cysteine-rich type 1 protein M130"
}